{
  "gene_symbol": "OOSP3",
  "gene": "UniProtKB:A0A2R8YFM6",
  "gene_name": "Oocyte-secreted protein 3",
  "term_id": "UNKNOWN:0001",
  "term_label": "Unknown molecular function"
}